{
  "term_label": "Unknown molecular function",
  "term_id": "UNKNOWN:0001",
  "gene_symbol": "LRP4",
  "gene": "UniProtKB:O75096",
  "gene_name": "Low-density lipoprotein receptor-related protein 4"
}